{
  "gene_symbol": "TMEM138",
  "term_id": "UNKNOWN:0001",
  "gene_name": "Transmembrane protein 138",
  "term_label": "Unknown molecular function",
  "gene": "UniProtKB:Q9NPI0"
}